{
  "gene_symbol": "RHBG",
  "term_label": "plasma membrane",
  "term_id": "GO:0005886",
  "gene": "UniProtKB:Q9H310",
  "gene_name": "Ammonium transporter Rh type B"
}